{
  "term_id": "GO:0000221",
  "gene_name": "V-type proton ATPase subunit C 1",
  "gene": "UniProtKB:P21283",
  "term_label": "vacuolar proton-transporting V-type ATPase, V1 domain",
  "gene_symbol": "ATP6V1C1"
}